{
  "term_label": "Unknown molecular function",
  "gene_symbol": "FAM204A",
  "gene_name": "Protein FAM204A",
  "gene": "UniProtKB:Q9H8W3",
  "term_id": "UNKNOWN:0001"
}